{
  "term_id": "UNKNOWN:0003",
  "term_label": "Unknown cellular component",
  "gene_symbol": "OR4F5",
  "gene": "UniProtKB:Q8NH21",
  "gene_name": "Olfactory receptor 4F5"
}